{
  "gene": "UniProtKB:Q8NHS4",
  "gene_name": "Clathrin heavy chain linker domain-containing protein 1",
  "gene_symbol": "CLHC1",
  "term_id": "UNKNOWN:0003",
  "term_label": "Unknown cellular component"
}